{
  "gene_symbol": "PRSS3P2",
  "gene": "UniProtKB:Q8NHM4",
  "gene_name": "Putative trypsin-6",
  "term_id": "GO:0005615",
  "term_label": "extracellular space"
}